{
  "term_id": "GO:0015629",
  "term_label": "actin cytoskeleton",
  "gene_name": "Transgelin-2",
  "gene_symbol": "TAGLN2",
  "gene": "UniProtKB:P37802"
}